sensory perception of fast pain [GO:0019234] (biological process) Definition: The series of events required for an organism to receive a fast pain stimulus, convert it to a molecular signal, and recognize and characterize the signal. This is a neurological process. Fast pain is often subjectively described as a sharp or stabbing pain; in humans, the signals from a fast pain stimulus are perceived and relayed along myelinated A-delta fibers to the central nervous system, reaching their target in about 0.1 seconds. Relationships: is a type of sensory perception of pain [GO:0019233] References: PMID:38704307